{
  "gene": "UniProtKB:Q9Y6H8",
  "term_id": "GO:0005922",
  "term_label": "connexin complex",
  "gene_name": "Gap junction alpha-3 protein",
  "gene_symbol": "GJA3"
}